{
  "gene_symbol": "PLCH1",
  "term_label": "phosphatidylinositol-4,5-bisphosphate phospholipase C activity",
  "gene": "UniProtKB:Q4KWH8",
  "gene_name": "1-phosphatidylinositol 4,5-bisphosphate phosphodiesterase eta-1",
  "term_id": "GO:0004435"
}